{
  "gene_symbol": "CLCA4",
  "gene_name": "Calcium-activated chloride channel regulator 4",
  "gene": "UniProtKB:Q14CN2",
  "term_id": "GO:0005886",
  "term_label": "plasma membrane"
}